{
  "gene": "UniProtKB:Q9UH77",
  "gene_symbol": "KLHL3",
  "term_id": "GO:0070294",
  "gene_name": "Kelch-like protein 3",
  "term_label": "renal sodium ion absorption"
}